dihydropyrimidine dehydrogenase (NAD+) complex [GO:0140690] (CC) Relationships: is a type of oxidoreductase complex [GO:1990204] Definition: A heteromultimeric complex capable of dihydropyrimidine dehydrogenase (NAD+); in E. coli, composed of PreA and PreT. References: PMID:21169495, PMID:34097066